{
  "term_id": "GO:0005634",
  "gene": "UniProtKB:P37231",
  "gene_symbol": "PPARG",
  "gene_name": "Peroxisome proliferator-activated receptor gamma",
  "term_label": "nucleus"
}